{
  "term_id": "GO:0019888",
  "gene_symbol": "PPP2R3A",
  "gene": "UniProtKB:Q06190",
  "term_label": "protein phosphatase regulator activity",
  "gene_name": "Serine_threonine-protein phosphatase 2A regulatory subunit B'' subunit alpha"
}